regulation of central B cell anergy [GO:0002914] (biological process) Subtypes: negative regulation of central B cell anergy [GO:0002915], positive regulation of central B cell anergy [GO:0002916] Definition: Any process that modulates the frequency, rate, or extent of central B cell anergy. Relationships: is a type of regulation of B cell anergy [GO:0002670]; is a type of regulation of central B cell tolerance induction [GO:0002895]; is_a regulation of B cell differentiation [GO:0045577]; regulates GO:0002341 Sources: GOC:add